negative regulation of gamma-delta T cell activation [GO:0046644] (biological process) Also known as: down regulation of gamma-delta T cell activation, down-regulation of gamma-delta T cell activation, downregulation of gamma-delta T cell activation, negative regulation of gamma-delta T lymphocyte activation, negative regulation of gamma-delta T-cell activation, negative regulation of gamma-delta T-lymphocyte activation, inhibition of gamma-delta T cell activation Definition: Any process that stops, prevents, or reduces the frequency, rate or extent of gamma-delta T cell activation. Sources: GOC:ai Subtypes: negative regulation of gamma-delta T cell differentiation [GO:0045587], GO:0046647, negative regulation of gamma-delta T cell activation involved in immune response [GO:2001192] Relationships: is a type of regulation of gamma-delta T cell activation [GO:0046643]; is a type of GO:0050868; negatively regulates GO:0046629